{
  "term_label": "endoplasmic reticulum membrane",
  "gene": "UniProtKB:Q9BSJ8",
  "gene_symbol": "ESYT1",
  "term_id": "GO:0005789",
  "gene_name": "Extended synaptotagmin-1"
}